{
  "term_label": "epidermal cell differentiation",
  "gene_name": "Transcription factor Ovo-like 2",
  "term_id": "GO:0009913",
  "gene": "UniProtKB:Q9BRP0",
  "gene_symbol": "OVOL2"
}